{
  "term_label": "tau protein binding",
  "gene": "UniProtKB:O00499",
  "gene_symbol": "BIN1",
  "gene_name": "Myc box-dependent-interacting protein 1",
  "term_id": "GO:0048156"
}